response to astaxanthin [GO:1905217] (biological process) Also known as: response to (3S,3'S)-3,3'-dihydroxy-beta,beta-carotene-4,4'-dione References: PMID:22309505 Sources: GOC:TermGenie, GO_REF:0000071 Relationships: is a type of response to lipid [GO:0033993] Definition: Any process that results in a change in state or activity of a cell or an organism (in terms of movement, secretion, enzyme production, gene expression, etc.) as a result of an astaxanthin stimulus. Subtypes: cellular response to astaxanthin [GO:1905218]